{
  "term_label": "protein serine/threonine kinase activity",
  "gene": "UniProtKB:Q8N752",
  "gene_name": "Casein kinase I isoform alpha-like",
  "term_id": "GO:0004674",
  "gene_symbol": "CSNK1A1L"
}